{
  "term_label": "actin filament",
  "gene_name": "Allograft inflammatory factor 1-like",
  "term_id": "GO:0005884",
  "gene": "UniProtKB:Q9BQI0",
  "gene_symbol": "AIF1L"
}